{
  "gene_name": "Profilin-2",
  "gene": "UniProtKB:P35080",
  "term_label": "cytoplasm",
  "term_id": "GO:0005737",
  "gene_symbol": "PFN2"
}